{
  "gene": "UniProtKB:Q6UWT4",
  "term_label": "Unknown cellular component",
  "gene_name": "Uncharacterized protein C5orf46",
  "gene_symbol": "C5orf46",
  "term_id": "UNKNOWN:0003"
}